monosaccharide metabolic process [GO:0005996] (biological process) Definition: The chemical reactions and pathways involving monosaccharides, the simplest carbohydrates. They are polyhydric alcohols containing either an aldehyde or a keto group and between three to ten or more carbon atoms. They form the constitutional repeating units of oligo- and polysaccharides. Sources: ISBN:0198506732 Also known as: monosaccharide metabolism Relationships: is a type of carbohydrate metabolic process [GO:0005975]; is a type of GO:0044281 Subtypes: hexose metabolic process [GO:0019318], pentose metabolic process [GO:0019321], L-ascorbic acid metabolic process [GO:0019852], tetrose metabolic process [GO:0033347], GO:0046364, monosaccharide catabolic process [GO:0046365], D-galacturonate metabolic process [GO:0046396]